gibberellin biosynthetic process [GO:0009686] (biological process) Definition: The chemical reactions and pathways resulting in the formation of gibberellin. Gibberellins are a class of highly modified terpenes that function as plant growth regulators. Subtypes: GO:0033470 Regulation: regulated by GO:0010371; positively regulated by positive regulation of gibberellin biosynthetic process [GO:0010372]; negatively regulated by negative regulation of gibberellin biosynthetic process [GO:0010373] Sources: ISBN:0387969845 Also known as: gibberellin biosynthesis, gibberellic acid anabolism, gibberellic acid biosynthesis, gibberellic acid biosynthetic process, gibberellic acid formation, gibberellic acid synthesis Relationships: is a type of gibberellin metabolic process [GO:0009685]; is a type of diterpenoid biosynthetic process [GO:0016102]; is a type of GO:0046394